corticospinal neuron axon guidance through the cerebral cortex [GO:0021967] (biological process) Relationships: is a type of axon guidance [GO:0007411]; is part of corticospinal neuron axon guidance [GO:0021966] References: PMID:9878731 Sources: GOC:cls, GOC:dgh, GOC:dph, GOC:jid, GO_REF:0000021 Definition: The process in which the migration of an axon growth cone of a pyramidal cell that is part of the corticospinal tract is directed from its cell body in layer V through the cerebral cortex in response to a combination of attractive and repulsive cues. Also known as: corticospinal neuron axon pathfinding through the cerebral cortex